{
  "gene_name": "Transmembrane protein 170B",
  "term_id": "GO:0090090",
  "gene_symbol": "TMEM170B",
  "gene": "UniProtKB:Q5T4T1",
  "term_label": "negative regulation of canonical Wnt signaling pathway"
}